{
  "gene": "UniProtKB:Q9P283",
  "term_id": "GO:0048675",
  "gene_symbol": "SEMA5B",
  "term_label": "axon extension",
  "gene_name": "Semaphorin-5B"
}